{
  "gene_symbol": "STRN4",
  "term_id": "GO:0090443",
  "gene_name": "Striatin-4",
  "gene": "UniProtKB:Q9NRL3",
  "term_label": "FAR/SIN/STRIPAK complex"
}